{
  "term_label": "embryonic skeletal system morphogenesis",
  "gene": "UniProtKB:P09016",
  "gene_symbol": "HOXD4",
  "term_id": "GO:0048704",
  "gene_name": "Homeobox protein Hox-D4"
}